cadherin binding involved in cell-cell adhesion [GO:0098641] (molecular function) Definition: Any cadherin binding that occurs as part of the process of cell-cell adhesion. Relationships: is a type of cadherin binding [GO:0045296]; is a type of cell-cell adhesion mediator activity [GO:0098632] Sources: GOC:dos